{
  "term_label": "RNA polymerase II transcription regulator complex",
  "gene_name": "Oxysterols receptor LXR-beta",
  "gene": "UniProtKB:P55055",
  "gene_symbol": "NR1H2",
  "term_id": "GO:0090575"
}